{
  "gene_symbol": "NDUFB6",
  "gene": "UniProtKB:O95139",
  "term_label": "Unknown molecular function",
  "term_id": "UNKNOWN:0001",
  "gene_name": "NADH dehydrogenase [ubiquinone] 1 beta subcomplex subunit 6"
}